11-cis retinal binding [GO:0005502] (molecular function) Also known as: vitamin A binding, 11-cis retinaldehyde binding, 11-cis-retinal binding Relationships: is a type of retinal binding [GO:0016918] Definition: Binding to 11-cis retinal, an isomer of retinal that plays an important role in the visual process in most vertebrates. 11-cis retinal combines with opsin in the rods (scotopsin) to form rhodopsin or visual purple. Retinal is one of the three compounds that makes up vitamin A. References: PMID:24403072